{
  "gene": "UniProtKB:Q969H9",
  "gene_name": "Disrupted in renal carcinoma protein 1",
  "term_label": "Unknown cellular component",
  "term_id": "UNKNOWN:0003",
  "gene_symbol": "DIRC1"
}